monopolar cell growth [GO:0042814] (biological process) Relationships: is a type of unidimensional cell growth [GO:0009826] Sources: GOC:vw Also known as: monopolar growth, monopolar cell elongation, polar cell elongation Definition: Polarized growth from one end of a cell. Regulation: regulated by regulation of monopolar cell growth [GO:0051513]; negatively regulated by negative regulation of monopolar cell growth [GO:0051514]; positively regulated by positive regulation of monopolar cell growth [GO:0051515]